{
  "gene_symbol": "TMEM115",
  "term_label": "Unknown molecular function",
  "gene_name": "Transmembrane protein 115",
  "term_id": "UNKNOWN:0001",
  "gene": "UniProtKB:Q12893"
}